{
  "gene_name": "Lysine-specific demethylase 4C",
  "term_label": "histone H3K36 demethylase activity",
  "gene": "UniProtKB:Q9H3R0",
  "gene_symbol": "KDM4C",
  "term_id": "GO:0051864"
}